{
  "gene_symbol": "CD1A",
  "term_id": "GO:0071723",
  "gene_name": "T-cell surface glycoprotein CD1a",
  "term_label": "lipopeptide binding",
  "gene": "UniProtKB:P06126"
}